{
  "term_label": "brain development",
  "gene": "UniProtKB:A8K0S8",
  "gene_name": "Putative homeobox protein Meis3-like 2",
  "gene_symbol": "MEIS3P2",
  "term_id": "GO:0007420"
}